{
  "term_label": "actomyosin structure organization",
  "gene": "UniProtKB:Q9HCS5",
  "gene_name": "Band 4.1-like protein 4A",
  "term_id": "GO:0031032",
  "gene_symbol": "EPB41L4A"
}